{
  "term_id": "UNKNOWN:0001",
  "gene": "UniProtKB:Q9BQQ3",
  "gene_symbol": "GORASP1",
  "term_label": "Unknown molecular function",
  "gene_name": "Golgi reassembly-stacking protein 1"
}